{
  "gene": "UniProtKB:Q9UKN1",
  "gene_symbol": "MUC12",
  "term_label": "Unknown biological process",
  "term_id": "UNKNOWN:0002",
  "gene_name": "Mucin-12"
}